{
  "gene_name": "T cell receptor alpha joining 31",
  "term_label": "Unknown cellular component",
  "gene": "UniProtKB:A0A075B700",
  "gene_symbol": "TRAJ31",
  "term_id": "UNKNOWN:0003"
}